{
  "gene": "UniProtKB:Q9BT81",
  "gene_name": "Transcription factor SOX-7",
  "gene_symbol": "SOX7",
  "term_id": "GO:0000978",
  "term_label": "RNA polymerase II cis-regulatory region sequence-specific DNA binding"
}